positive regulation of somatic muscle development [GO:0062224] (biological process) Relationships: is a type of positive regulation of developmental process [GO:0051094]; is a type of regulation of somatic muscle development [GO:0062223]; positively regulates GO:0007525 Definition: Any process that increases the rate, frequency or extent of somatic muscle development. Subtypes: positive regulation of adult somatic muscle development [GO:0062227], positive regulation of larval somatic muscle development [GO:0062231] References: PMID:16643882, PMID:25758712